homeostasis of number of retina cells [GO:0048877] (biological process) Definition: Any biological process involved in the maintenance of the steady-state number of cells within a population of cells in the retina. Relationships: is a type of retina homeostasis [GO:0001895]; is a type of homeostasis of number of cells within a tissue [GO:0048873] Sources: GOC:dph, GOC:isa_complete, GOC:tb